{
  "term_label": "Unknown molecular function",
  "term_id": "UNKNOWN:0001",
  "gene": "UniProtKB:Q07627",
  "gene_symbol": "KRTAP1-1",
  "gene_name": "Keratin-associated protein 1-1"
}